miRNA processing [GO:0035196] (biological process) References: PMID:15066275, PMID:15066283, PMID:23985560, PMID:28379604 Sources: GOC:aruk, GOC:bc, GOC:dph, GOC:rl, GOC:tb Relationships: is a type of regulatory ncRNA processing [GO:0070918] Also known as: miRNA biosynthetic process, microRNA biosynthesis, microRNA biosynthetic process, microRNA metabolic process, microRNA metabolism, gene silencing by miRNA, production of miRNAs, miRNA maturation, miRNA-mediated gene silencing, production of miRNAs, microRNA biogenesis, microRNA processing, microRNA-mediated gene silencing, production of microRNAs, production of miRNAs involved in gene silencing by miRNA, production of microRNAs involved in gene silencing by microRNA, miRNA biogenesis Subtypes: primary miRNA processing [GO:0031053], pre-miRNA processing [GO:0031054] Regulation: RO_0002211 by regulation of miRNA processing [GO:1903798]; negatively regulated by negative regulation of miRNA processing [GO:1903799]; positively regulated by positive regulation of miRNA processing [GO:1903800] Definition: A process leading to the generation of a functional miRNA. Includes the cleavage of stem-loop RNA precursors into microRNAs (miRNAs). miRNAs are a class of small RNAs that primarily silence genes by blocking the translation of mRNA transcripts into protein, or by increasing the degradation of non-protein-coding RNA transcripts.